{
  "gene": "UniProtKB:O96000",
  "gene_symbol": "NDUFB10",
  "gene_name": "NADH dehydrogenase [ubiquinone] 1 beta subcomplex subunit 10",
  "term_label": "Unknown molecular function",
  "term_id": "UNKNOWN:0001"
}